{
  "term_label": "cytoplasm",
  "gene_symbol": "CAPN3",
  "term_id": "GO:0005737",
  "gene_name": "Calpain-3",
  "gene": "UniProtKB:P20807"
}